{
  "gene": "UniProtKB:Q86V40",
  "gene_name": "Metalloprotease TIKI1",
  "term_label": "Unknown biological process",
  "gene_symbol": "TRABD2A",
  "term_id": "UNKNOWN:0002"
}